{
  "term_label": "positive regulation of phosphatidylinositol 3-kinase/protein kinase B signal transduction",
  "term_id": "GO:0051897",
  "gene_symbol": "TEK",
  "gene_name": "Angiopoietin-1 receptor",
  "gene": "UniProtKB:Q02763"
}